{
  "gene_name": "FGGY carbohydrate kinase domain-containing protein",
  "term_label": "cytoplasm",
  "gene": "UniProtKB:Q96C11",
  "gene_symbol": "FGGY",
  "term_id": "GO:0005737"
}